{
  "term_label": "nucleus",
  "gene_symbol": "HES3",
  "gene_name": "Transcription factor HES-3",
  "term_id": "GO:0005634",
  "gene": "UniProtKB:Q5TGS1"
}